{
  "gene": "UniProtKB:A0A087X0K7",
  "term_id": "GO:0007166",
  "gene_name": "Probable non-functional T cell receptor beta variable 17",
  "term_label": "cell surface receptor signaling pathway",
  "gene_symbol": "TRBV17"
}